{
  "gene_symbol": "PDZD9",
  "term_id": "UNKNOWN:0001",
  "gene": "UniProtKB:Q8IXQ8",
  "gene_name": "PDZ domain-containing protein 9",
  "term_label": "Unknown molecular function"
}